{
  "term_label": "bicarbonate transport",
  "term_id": "GO:0015701",
  "gene_symbol": "SLC4A10",
  "gene_name": "Sodium-driven chloride bicarbonate exchanger",
  "gene": "UniProtKB:Q6U841"
}